{
  "gene": "UniProtKB:Q8WWW8",
  "gene_name": "GRB2-associated-binding protein 3",
  "term_id": "GO:0007165",
  "term_label": "signal transduction",
  "gene_symbol": "GAB3"
}